regulation of cardiac neural crest cell migration involved in outflow tract morphogenesis [GO:1905310] (biological process) References: PMID:17628518 Sources: GOC:BHF, GOC:TermGenie, GOC:rl, GO_REF:0000058 Definition: Any process that modulates the frequency, rate or extent of cardiac neural crest cell migration involved in outflow tract morphogenesis. Subtypes: GO:1905311, GO:1905312 Relationships: is a type of GO:0030334; regulates cardiac neural crest cell migration involved in outflow tract morphogenesis [GO:0003253]